{
  "term_id": "GO:0006888",
  "gene": "UniProtKB:Q9BRL7",
  "gene_symbol": "SEC22C",
  "term_label": "endoplasmic reticulum to Golgi vesicle-mediated transport",
  "gene_name": "Vesicle-trafficking protein SEC22c"
}